{
  "term_id": "GO:0005634",
  "gene_name": "Upstream-binding factor 1-like protein 1",
  "gene_symbol": "UBTFL1",
  "gene": "UniProtKB:P0CB47",
  "term_label": "nucleus"
}